{
  "gene_name": "Olfactory receptor 1L4",
  "gene_symbol": "OR1L4",
  "gene": "UniProtKB:Q8NGR5",
  "term_label": "signal transduction",
  "term_id": "GO:0007165"
}